{
  "gene": "UniProtKB:Q5BJH7",
  "gene_symbol": "YIF1B",
  "gene_name": "Protein YIF1B",
  "term_id": "UNKNOWN:0001",
  "term_label": "Unknown molecular function"
}